{
  "term_label": "cytoplasmic vesicle",
  "gene": "UniProtKB:Q8N8V2",
  "gene_symbol": "GBP7",
  "gene_name": "Guanylate-binding protein 7",
  "term_id": "GO:0031410"
}